{
  "gene": "UniProtKB:Q9BXE9",
  "gene_name": "Vomeronasal type-1 receptor 3",
  "term_id": "GO:0005886",
  "term_label": "plasma membrane",
  "gene_symbol": "VN1R3"
}